{
  "gene_symbol": "PLB1",
  "gene": "UniProtKB:Q6P1J6",
  "term_label": "phosphatidylcholine lysophospholipase activity",
  "term_id": "GO:0004622",
  "gene_name": "Phospholipase B1, membrane-associated"
}